positive regulation of dendrite morphogenesis [GO:0050775] (biological process) Sources: GOC:ai Relationships: is_a positive regulation of cell morphogenesis [GO:0010770]; is a type of positive regulation of cell projection organization [GO:0031346]; is_a regulation of dendrite morphogenesis [GO:0048814]; is a type of GO:0050769; RO_0002213 dendrite morphogenesis [GO:0048813] Also known as: up regulation of dendrite morphogenesis, up-regulation of dendrite morphogenesis, upregulation of dendrite morphogenesis, activation of dendrite morphogenesis, stimulation of dendrite morphogenesis Definition: Any process that activates or increases the frequency, rate or extent of dendrite morphogenesis. Subtypes: GO:0061003